{
  "term_id": "GO:0003697",
  "gene_name": "Nuclear ubiquitous casein and cyclin-dependent kinase substrate 1",
  "term_label": "single-stranded DNA binding",
  "gene": "UniProtKB:Q9H1E3",
  "gene_symbol": "NUCKS1"
}